{
  "term_label": "molecular adaptor activity",
  "term_id": "GO:0060090",
  "gene_symbol": "AKAP5",
  "gene": "UniProtKB:P24588",
  "gene_name": "A-kinase anchor protein 5"
}